{
  "gene_name": "Small ribosomal subunit protein eS8",
  "gene_symbol": "RPS8",
  "gene": "UniProtKB:P62241",
  "term_label": "cytosolic small ribosomal subunit",
  "term_id": "GO:0022627"
}